{
  "gene": "UniProtKB:O75676",
  "term_label": "regulation of DNA-templated transcription",
  "gene_name": "Ribosomal protein S6 kinase alpha-4",
  "gene_symbol": "RPS6KA4",
  "term_id": "GO:0006355"
}